{
  "gene_symbol": "RAG2",
  "term_id": "GO:0097519",
  "gene": "UniProtKB:P55895",
  "term_label": "DNA recombinase complex",
  "gene_name": "V(D)J recombination-activating protein 2"
}